7-dehydrocholesterol reductase activity [GO:0047598] (molecular function) Relationships: is a type of oxidoreductase activity, acting on the CH-CH group of donors, NAD or NADP as acceptor [GO:0016628] Sources: RHEA:23984 Definition: Catalysis of the reaction: cholesterol + NADP+ = 7-dehydrocholesterol + H+ + NADPH. Also known as: sterol Delta(7)-reductase activity, 7-DHC reductase activity, cholesterol:NADP+ delta7-oxidoreductase activity, sterol delta7-reductase activity